positive regulation of cortisol secretion [GO:0051464] (biological process) Definition: Any process that activates or increases the frequency, rate or extent of the regulated release of cortisol from a cell. Sources: GOC:ai Also known as: up regulation of cortisol secretion, up-regulation of cortisol secretion, upregulation of cortisol secretion, activation of cortisol secretion, stimulation of cortisol secretion Relationships: is a type of regulation of cortisol secretion [GO:0051462]; is a type of positive regulation of glucocorticoid secretion [GO:2000851]; positively regulates GO:0043400